positive regulation of inflammatory response [GO:0050729] (BP) Relationships: is a type of positive regulation of defense response [GO:0031349]; is a type of positive regulation of response to external stimulus [GO:0032103]; is a type of regulation of inflammatory response [GO:0050727]; positively regulates inflammatory response [GO:0006954] Subtypes: GO:0002675, positive regulation of chronic inflammatory response [GO:0002678], positive regulation of inflammatory response to antigenic stimulus [GO:0002863], GO:0035491, positive regulation of respiratory burst involved in inflammatory response [GO:0060265], GO:0106016, GO:0140639, positive regulation of neuroinflammatory response [GO:0150078], positive regulation of histamine secretion by mast cell [GO:1903595] Definition: Any process that activates or increases the frequency, rate or extent of the inflammatory response. Sources: GOC:ai Also known as: up regulation of inflammatory response, up-regulation of inflammatory response, upregulation of inflammatory response, activation of inflammatory response, stimulation of inflammatory response